{
  "term_id": "GO:0036337",
  "gene_symbol": "CASP8AP2",
  "term_label": "Fas signaling pathway",
  "gene_name": "CASP8-associated protein 2",
  "gene": "UniProtKB:Q9UKL3"
}